A-type (transient outward) potassium channel activity [GO:0005250] (molecular function) References: PMID:5575340 Sources: GOC:mah Definition: Enables the transmembrane transfer of a potassium ion by an outwardly-rectifying voltage-gated channel that produces a transient outward current upon a step change in membrane potential. Relationships: is a type of outward rectifier potassium channel activity [GO:0015271]